{
  "gene_symbol": "GEMIN8",
  "term_label": "spliceosomal snRNP assembly",
  "gene": "UniProtKB:Q9NWZ8",
  "term_id": "GO:0000387",
  "gene_name": "Gem-associated protein 8"
}